symbiont-mediated suppression of host phagosome acidification [GO:0141159] (biological process) References: PMID:20333253, PMID:22087003, PMID:33505976 Relationships: is a type of symbiont-mediated perturbation of host defense response [GO:0052031] Definition: A process in which a symbiont inhibits or disrupts the normal acidification of host phagosomes. Mechanisms by which a symbiont prevents host phagosome acidification include the inhibitition of host V-ATPase, the proton pump that acidifies the phagosome, or disruption of the phagosome membrane by pore-forming toxin. The host is defined as the larger of the organisms involved in a symbiotic interaction.